cellular response to cholecystokinin [GO:0061848] (biological process) Definition: Any process that results in a change in state or activity of a cell (in terms of movement, secretion, enzyme production, gene expression, etc.) as a result of a cholecystokinin stimulus. Relationships: is_a response to cholecystokinin [GO:0061847]; is a type of cellular response to peptide hormone stimulus [GO:0071375] References: PMID:14622258